basal part of cell [GO:0045178] (cellular component) Relationships: is a type of cellular anatomical structure [GO:0110165] Sources: GOC:mah, ISBN:0815316194 Definition: The region of a cell situated near the base. For example, in a polarized epithelial cell, the basal surface rests on the basal lamina that separates the epithelium from other tissue.